{
  "term_label": "Unknown cellular component",
  "gene_symbol": "IRGQ",
  "term_id": "UNKNOWN:0003",
  "gene": "UniProtKB:Q8WZA9",
  "gene_name": "Immunity-related GTPase family Q protein"
}